{
  "gene_name": "Putative transmembrane protein CXorf1",
  "term_label": "Unknown biological process",
  "term_id": "UNKNOWN:0002",
  "gene": "UniProtKB:O96002",
  "gene_symbol": "CXorf1"
}